{
  "term_label": "nucleus",
  "gene": "UniProtKB:Q9Y6F8",
  "term_id": "GO:0005634",
  "gene_name": "Testis-specific chromodomain protein Y 1",
  "gene_symbol": "CDY1B"
}